{
  "gene_name": "Disintegrin and metalloproteinase domain-containing protein 15",
  "term_label": "proteolysis",
  "gene": "UniProtKB:Q13444",
  "gene_symbol": "ADAM15",
  "term_id": "GO:0006508"
}